{
  "term_label": "oxygen transport",
  "gene_symbol": "HBG2",
  "gene_name": "Hemoglobin subunit gamma-2",
  "gene": "UniProtKB:P69892",
  "term_id": "GO:0015671"
}